{
  "gene_name": "Cyclin-I2",
  "term_id": "GO:0016538",
  "gene_symbol": "CCNI2",
  "gene": "UniProtKB:Q6ZMN8",
  "term_label": "cyclin-dependent protein serine/threonine kinase regulator activity"
}